negative regulation of protein localization to presynapse [GO:1905385] (biological process) Also known as: down regulation of protein localisation in presynapse, down regulation of protein localisation to presynapse, down regulation of protein localization in presynapse, down regulation of protein localization to presynapse, down regulation of recruitment of presynaptic proteins, down-regulation of protein localisation in presynapse, down-regulation of protein localisation to presynapse, down-regulation of protein localization in presynapse, down-regulation of protein localization to presynapse, down-regulation of recruitment of presynaptic proteins, downregulation of protein localisation in presynapse, downregulation of protein localisation to presynapse, downregulation of protein localization in presynapse, downregulation of protein localization to presynapse, downregulation of recruitment of presynaptic proteins, negative regulation of protein localisation in presynapse, negative regulation of protein localisation to presynapse, negative regulation of protein localization in presynapse, negative regulation of recruitment of presynaptic proteins, inhibition of protein localisation in presynapse, inhibition of protein localisation to presynapse, inhibition of protein localization in presynapse, inhibition of protein localization to presynapse, inhibition of recruitment of presynaptic proteins References: PMID:24449494 Sources: GOC:PARL, GOC:TermGenie, GOC:bf, GO_REF:0000058 Definition: Any process that stops, prevents or reduces the frequency, rate or extent of protein localization to presynapse. Relationships: is a type of negative regulation of protein localization [GO:1903828]; is a type of GO:1905384; negatively regulates GO:1905383